{
  "term_id": "GO:0015279",
  "term_label": "store-operated calcium channel activity",
  "gene_symbol": "ORAI2",
  "gene": "UniProtKB:Q96SN7",
  "gene_name": "Protein orai-2"
}